{
  "gene_symbol": "TFAP2C",
  "term_id": "GO:0000977",
  "term_label": "RNA polymerase II transcription regulatory region sequence-specific DNA binding",
  "gene_name": "Transcription factor AP-2 gamma",
  "gene": "UniProtKB:Q92754"
}